detection of folic acid [GO:0031318] (biological process) Definition: The series of events in which a folic acid stimulus is received by a cell and converted into a molecular signal. Relationships: is a type of detection of nutrient [GO:0009594]; is a type of response to folic acid [GO:0051593] Also known as: detection of folate, folate detection, folate sensing, folic acid detection, folic acid sensing Sources: GOC:pg